lysobisphosphatidic acid biosynthetic process [GO:2001312] (biological process) Relationships: is a type of glycerophospholipid biosynthetic process [GO:0046474]; is a type of GO:1901137; is a type of GO:2001311 Definition: The chemical reactions and pathways resulting in the formation of a lysobisphosphatidic acid. A lysobisphosphatidic acid is a lysophosphatidic acid having the unusual property of a phosphodiester moiety linked to positions sn-1 and sn1' of glycerol; and two additional fatty acids esterified to the glycerol head group. Also known as: LBPA anabolism, LBPA biosynthesis, LBPA biosynthetic process, LBPA formation, LBPA synthesis, bis(monoacylglycerol) hydrogen phosphate (BMP) anabolism, bis(monoacylglycerol) hydrogen phosphate (BMP) biosynthesis, bis(monoacylglycerol) hydrogen phosphate (BMP) biosynthetic process, bis(monoacylglycerol) hydrogen phosphate (BMP) formation, bis(monoacylglycerol) hydrogen phosphate (BMP) synthesis, bis(monoacylglycerol) hydrogen phosphate anabolism, bis(monoacylglycerol) hydrogen phosphate biosynthesis, bis(monoacylglycerol) hydrogen phosphate biosynthetic process, bis(monoacylglycerol) hydrogen phosphate formation, bis(monoacylglycerol) hydrogen phosphate synthesis, lysobisphosphatidic acid anabolism, lysobisphosphatidic acid biosynthesis, lysobisphosphatidic acid formation, lysobisphosphatidic acid synthesis Sources: GOC:mw